{
  "gene": "UniProtKB:P35914",
  "gene_symbol": "HMGCL",
  "gene_name": "Hydroxymethylglutaryl-CoA lyase, mitochondrial",
  "term_id": "GO:0006552",
  "term_label": "L-leucine catabolic process"
}